{
  "gene_symbol": "ACKR1",
  "gene": "UniProtKB:Q16570",
  "gene_name": "Atypical chemokine receptor 1",
  "term_label": "C-C chemokine binding",
  "term_id": "GO:0019957"
}